{
  "gene": "UniProtKB:P62316",
  "gene_symbol": "SNRPD2",
  "term_label": "U1 snRNP",
  "term_id": "GO:0005685",
  "gene_name": "Small nuclear ribonucleoprotein Sm D2"
}